{
  "term_id": "GO:0000978",
  "gene_name": "Nuclear receptor subfamily 2 group F member 6",
  "term_label": "RNA polymerase II cis-regulatory region sequence-specific DNA binding",
  "gene": "UniProtKB:P10588",
  "gene_symbol": "NR2F6"
}